{
  "gene_symbol": "DLX6",
  "term_label": "regulation of transcription by RNA polymerase II",
  "gene": "UniProtKB:P56179",
  "term_id": "GO:0006357",
  "gene_name": "Homeobox protein DLX-6"
}